{
  "gene_symbol": "GRIA3",
  "gene": "UniProtKB:P42263",
  "gene_name": "Glutamate receptor 3",
  "term_label": "AMPA glutamate receptor complex",
  "term_id": "GO:0032281"
}